{
  "gene": "UniProtKB:P23528",
  "term_label": "cytoplasm",
  "gene_name": "Cofilin-1",
  "gene_symbol": "CFL1",
  "term_id": "GO:0005737"
}